{
  "gene": "UniProtKB:P09486",
  "term_id": "GO:0050807",
  "gene_name": "SPARC",
  "term_label": "regulation of synapse organization",
  "gene_symbol": "SPARC"
}